{
  "gene": "UniProtKB:O75069",
  "gene_name": "Transmembrane and coiled-coil domains protein 2",
  "gene_symbol": "TMCC2",
  "term_id": "GO:0012505",
  "term_label": "endomembrane system"
}